{
  "gene": "UniProtKB:Q9UBX0",
  "term_label": "DNA-binding transcription repressor activity, RNA polymerase II-specific",
  "gene_symbol": "HESX1",
  "gene_name": "Homeobox expressed in ES cells 1",
  "term_id": "GO:0001227"
}